{
  "gene_symbol": "UTS2B",
  "gene": "UniProtKB:Q765I0",
  "gene_name": "Urotensin-2B",
  "term_label": "Unknown cellular component",
  "term_id": "UNKNOWN:0003"
}